L-lysine:L-arginine antiporter activity [GO:0106439] (MF) Note: L-arginine:L-lysine antiporter activity Definition: Enables the transfer of a solute or solutes from one side of a membrane to the other according to the reaction: L-lysine(out) + L-arginine(in) = L-lysine(in) + L-arginine(out). References: PMID:10903140 Sources: RHEA:70827 Relationships: is_a L-lysine transmembrane transporter activity [GO:0015189]; is a type of antiporter activity [GO:0015297]; is a type of L-arginine transmembrane transporter activity [GO:0061459]